{
  "gene_symbol": "USP42",
  "gene_name": "Ubiquitin carboxyl-terminal hydrolase 42",
  "term_id": "GO:0005829",
  "gene": "UniProtKB:Q9H9J4",
  "term_label": "cytosol"
}